{
  "term_id": "GO:0000245",
  "gene_symbol": "SRPK1",
  "term_label": "spliceosomal complex assembly",
  "gene": "UniProtKB:Q96SB4",
  "gene_name": "SRSF protein kinase 1"
}